positive regulation of granulosa cell apoptotic process [GO:1904710] (biological process) Definition: Any process that activates or increases the frequency, rate or extent of granulosa cell apoptotic process. References: PMID:19208546 Sources: GOC:TermGenie, GO_REF:0000058 Also known as: positive regulation of granulosa cell of ovary apoptotic process, up regulation of granulosa cell apoptotic process, up regulation of granulosa cell of ovary apoptotic process, up-regulation of granulosa cell apoptotic process, up-regulation of granulosa cell of ovary apoptotic process, upregulation of granulosa cell apoptotic process, upregulation of granulosa cell of ovary apoptotic process, activation of granulosa cell apoptosis, activation of granulosa cell apoptotic process, activation of granulosa cell of ovary apoptosis, activation of granulosa cell of ovary apoptotic process, positive regulation of granulosa cell apoptosis, positive regulation of granulosa cell of ovary apoptosis, up regulation of granulosa cell apoptosis, up regulation of granulosa cell of ovary apoptosis, up-regulation of granulosa cell apoptosis, up-regulation of granulosa cell of ovary apoptosis, upregulation of granulosa cell apoptosis, upregulation of granulosa cell of ovary apoptosis Relationships: is a type of positive regulation of epithelial cell apoptotic process [GO:1904037]; is a type of GO:1904708; positively regulates granulosa cell apoptotic process [GO:1904700]